ortho-trichlorophenol reductive dehalogenase activity [GO:0050781] (molecular function) References: PMID:12697029 Sources: GOC:ai Relationships: is a type of oxidoreductase activity [GO:0016491] Definition: Catalysis of the reaction: 2,4,6-trichlorophenol + 2 H+ + 2 e- = 2,4-dichlorophenol + HCl. Also known as: 2,4,6-TCP reductive dehalogenase activity, 2,4,6-trichlorophenol reductive dehalogenase activity